{
  "gene_symbol": "SPACA9",
  "gene_name": "Sperm acrosome-associated protein 9",
  "term_id": "UNKNOWN:0001",
  "gene": "UniProtKB:Q96E40",
  "term_label": "Unknown molecular function"
}